{
  "gene_symbol": "RRM2",
  "term_id": "GO:0004748",
  "gene_name": "Ribonucleoside-diphosphate reductase subunit M2",
  "term_label": "ribonucleoside-diphosphate reductase activity, thioredoxin disulfide as acceptor",
  "gene": "UniProtKB:P31350"
}